{
  "gene": "UniProtKB:Q6P4F2",
  "term_id": "GO:0005739",
  "gene_name": "Ferredoxin-2, mitochondrial",
  "gene_symbol": "FDX2",
  "term_label": "mitochondrion"
}